positive regulation of C-C chemokine receptor CCR7 signaling pathway [GO:1903082] (biological process) Relationships: is a type of positive regulation of chemokine-mediated signaling pathway [GO:0070101]; is a type of GO:1903080; positively regulates C-C chemokine receptor CCR7 signaling pathway [GO:0038118] Also known as: positive regulation of C-C chemokine receptor CCR7 signalling pathway, up regulation of C-C chemokine receptor CCR7 signaling pathway, up regulation of C-C chemokine receptor CCR7 signalling pathway, up-regulation of C-C chemokine receptor CCR7 signaling pathway, up-regulation of C-C chemokine receptor CCR7 signalling pathway, upregulation of C-C chemokine receptor CCR7 signaling pathway, upregulation of C-C chemokine receptor CCR7 signalling pathway, activation of C-C chemokine receptor CCR7 signaling pathway, activation of C-C chemokine receptor CCR7 signalling pathway, activation of CCR7 signaling pathway, positive regulation of CCR7 signaling pathway, up regulation of CCR7 signaling pathway, up-regulation of CCR7 signaling pathway, upregulation of CCR7 signaling pathway Definition: Any process that activates or increases the frequency, rate or extent of C-C chemokine receptor CCR7 signaling pathway. References: PMID:11602640 Sources: GOC:BHF, GOC:TermGenie, GOC:rl, GO_REF:0000058